{
  "gene_name": "FYVE, RhoGEF and PH domain-containing protein 5",
  "term_id": "GO:0005085",
  "gene_symbol": "FGD5",
  "gene": "UniProtKB:Q6ZNL6",
  "term_label": "guanyl-nucleotide exchange factor activity"
}